{
  "gene": "UniProtKB:Q3KNW5",
  "term_label": "bile acid:sodium symporter activity",
  "gene_name": "Sodium-dependent organic anion transporter",
  "term_id": "GO:0008508",
  "gene_symbol": "SLC10A6"
}